{
  "gene": "UniProtKB:O60763",
  "gene_name": "General vesicular transport factor p115",
  "gene_symbol": "USO1",
  "term_id": "GO:0005783",
  "term_label": "endoplasmic reticulum"
}